{
  "gene": "UniProtKB:Q2M3G4",
  "term_id": "GO:0043296",
  "gene_symbol": "SHROOM1",
  "term_label": "apical junction complex",
  "gene_name": "Protein Shroom1"
}